{
  "gene_name": "Dynein axonemal intermediate chain 4",
  "term_id": "GO:0003341",
  "gene_symbol": "DNAI4",
  "term_label": "cilium movement",
  "gene": "UniProtKB:Q5VTH9"
}